{
  "gene": "UniProtKB:Q96BK5",
  "term_label": "Unknown biological process",
  "term_id": "UNKNOWN:0002",
  "gene_name": "PIN2_TERF1-interacting telomerase inhibitor 1",
  "gene_symbol": "PINX1"
}